specification of connecting tubule identity [GO:0072085] (biological process) Subtypes: specification of mesonephric connecting tubule identity [GO:0061281], specification of metanephric connecting tubule identity [GO:0072294] Relationships: is a type of specification of nephron tubule identity [GO:0072081]; is part of connecting tubule development [GO:0072027] Definition: The process in which the connecting tubule of the kidney nephron acquires its identity. Sources: GOC:bf, GOC:mtg_kidney_jan10